{
  "term_id": "GO:0005739",
  "gene": "UniProtKB:Q9BZJ4",
  "gene_symbol": "SLC25A39",
  "gene_name": "Probable mitochondrial glutathione transporter SLC25A39",
  "term_label": "mitochondrion"
}